{
  "term_label": "DNA-binding transcription factor activity, RNA polymerase II-specific",
  "gene": "UniProtKB:P35548",
  "gene_symbol": "MSX2",
  "gene_name": "Homeobox protein MSX-2",
  "term_id": "GO:0000981"
}